mineralocorticoid metabolic process [GO:0008212] (biological process) Relationships: is a type of steroid metabolic process [GO:0008202]; is a type of hormone metabolic process [GO:0042445] Sources: ISBN:0198506732 Definition: The chemical reactions and pathways involving mineralocorticoids, hormonal C21 corticosteroids synthesized from cholesterol. Mineralocorticoids act primarily on water and electrolyte balance. Subtypes: mineralocorticoid biosynthetic process [GO:0006705], mineralocorticoid catabolic process [GO:0006712], aldosterone metabolic process [GO:0032341] Also known as: mineralocorticoid metabolism